seed oilbody biogenesis [GO:0010344] (biological process) Definition: A cellular process that results in the biosynthesis of constituent macromolecules, assembly, and arrangement of constituent parts of a seed oilbody. Seed oilbodies are simple organelles comprising a matrix of triglyceride surrounded by a phospholipid monolayer embedded and covered with unique proteins called oleosins. Seed oilbodies supply the energy requirements for the growth of the seedling after germination. Relationships: is a type of GO:0044085; is part of seed development [GO:0048316] Also known as: seed oil body organization, oleosome biogenesis, spherosome biogenesis References: PMID:16877495 Sources: GOC:jl